{
  "gene_name": "Homeobox protein Hox-C9",
  "term_label": "proximal/distal pattern formation",
  "term_id": "GO:0009954",
  "gene_symbol": "HOXC9",
  "gene": "UniProtKB:P31274"
}